melanin biosynthetic process from tyrosine [GO:0006583] (biological process) Definition: The chemical reactions and pathways resulting in the formation of melanin from other compounds, including tyrosine. Also known as: melanin anabolism from tyrosine, melanin formation from tyrosine, melanin synthesis from tyrosine Sources: GOC:go_curators Relationships: is a type of tyrosine metabolic process [GO:0006570]; is a type of melanin biosynthetic process [GO:0042438]